TORC1 complex [GO:0031931] (cellular component) Also known as: TOR complex 1, TORC 1 complex, TORC1, nutrient sensitive complex, rapamycin and nutrient-sensitive TOR complex, dTOR/dRaptor complex, dTORC1, mTORC1 Relationships: is a type of TOR complex [GO:0038201] Definition: A protein complex that contains at least TOR (target of rapamycin) and Raptor (regulatory-associated protein of TOR), or orthologs of, in complex with other signaling components. Mediates the phosphorylation and activation of S6K. In Saccharomyces, the complex contains Kog1p, Lst8p, Tco89p, and either Tor1p or Tor2p. References: PMID:15780592, PMID:16469695, PMID:21548787 Sources: GOC:jh